cytokinesis [GO:0000910] (biological process) Regulation: regulated by regulation of cytokinesis [GO:0032465]; negatively regulated by negative regulation of cytokinesis [GO:0032466]; positively regulated by positive regulation of cytokinesis [GO:0032467] Definition: The division of the cytoplasm and the plasma membrane of a cell and its partitioning into two daughter cells. Also known as: cell cycle cytokinesis, cytokinesis involved in cell cycle Note: Note that this term should not be used for direct annotation. When annotating eukaryotic species, mitotic or meiotic cytokinesis should always be specified for manual annotation and for prokaryotic species use 'FtsZ-dependent cytokinesis ; GO:0043093' or Cdv-dependent cytokinesis ; GO:0061639. Also, note that cytokinesis does not necessarily result in physical separation and detachment of the two daughter cells from each other. Subtypes: GO:0000911, FtsZ-dependent cytokinesis [GO:0043093], Cdv-dependent cytokinesis [GO:0061639], cytoskeleton-dependent cytokinesis [GO:0061640] Relationships: is a type of cell cycle process [GO:0022402]; is part of cell division [GO:0051301]; has part membrane fission [GO:0090148] Sources: GOC:mtg_cell_cycle